{
  "term_label": "membrane",
  "gene_name": "Oxysterol-binding protein-related protein 5",
  "gene": "UniProtKB:Q9H0X9",
  "term_id": "GO:0016020",
  "gene_symbol": "OSBPL5"
}